non-lytic viral release [GO:0046753] (biological process) Definition: The exit of a viral particle from a host cell that does not involve cell lysis. Sources: GOC:bf, GOC:jl, ISBN:0072370319 Relationships: is a type of viral release from host cell [GO:0019076] Subtypes: viral exocytosis [GO:0046754], viral budding from plasma membrane [GO:0046761], GO:0099045